{
  "gene_name": "Lipid transferase CIDEA",
  "term_label": "lipid transfer activity",
  "term_id": "GO:0120013",
  "gene_symbol": "CIDEA",
  "gene": "UniProtKB:O60543"
}